beta-galactoside alpha-2,3-sialyltransferase activity [GO:0052798] (molecular function) Definition: Catalysis of the transfer of sialyl residues alpha-2,3-linked to a beta galactosyl residue on the donor to form an alpha-2,3 linkage to a terminal beta galactosyl residue on the acceptor. Relationships: is a type of sialyltransferase activity [GO:0008373] References: PMID:7826016, PMID:8405811 Sources: GOC:mengo_curators Also known as: trans-sialidase activity